{
  "gene_name": "Olfactory receptor 5D13",
  "gene_symbol": "OR5D13",
  "term_label": "odorant binding",
  "gene": "UniProtKB:Q8NGL4",
  "term_id": "GO:0005549"
}